{
  "term_label": "extracellular region",
  "gene_name": "Fetuin-B",
  "gene_symbol": "FETUB",
  "term_id": "GO:0005576",
  "gene": "UniProtKB:Q9UGM5"
}